{
  "gene_name": "Adenylyltransferase and sulfurtransferase MOCS3",
  "term_id": "GO:0032447",
  "gene": "UniProtKB:O95396",
  "term_label": "protein urmylation",
  "gene_symbol": "MOCS3"
}